{
  "gene_symbol": "TMPPE",
  "gene": "UniProtKB:Q6ZT21",
  "term_id": "UNKNOWN:0001",
  "term_label": "Unknown molecular function",
  "gene_name": "Transmembrane protein with metallophosphoesterase domain"
}